{
  "gene_name": "Histatin-3",
  "gene": "UniProtKB:P15516",
  "term_label": "Unknown molecular function",
  "term_id": "UNKNOWN:0001",
  "gene_symbol": "HTN3"
}